{
  "gene": "UniProtKB:Q0VFX4",
  "gene_name": "Putative uncharacterized protein LOC100128554",
  "term_id": "UNKNOWN:0001",
  "term_label": "Unknown molecular function",
  "gene_symbol": "Q0VFX4"
}